{
  "gene_symbol": "RSRC1",
  "term_label": "alternative mRNA splicing, via spliceosome",
  "term_id": "GO:0000380",
  "gene_name": "Serine_Arginine-related protein 53",
  "gene": "UniProtKB:Q96IZ7"
}